{
  "gene_name": "Laminin subunit alpha-4",
  "term_label": "signal transduction",
  "gene": "UniProtKB:Q16363",
  "gene_symbol": "LAMA4",
  "term_id": "GO:0007165"
}